{
  "gene_symbol": "BLOC1S4",
  "term_id": "UNKNOWN:0002",
  "gene_name": "Biogenesis of lysosome-related organelles complex 1 subunit 4",
  "gene": "UniProtKB:Q9NUP1",
  "term_label": "Unknown biological process"
}